{
  "term_label": "nucleoside diphosphate kinase activity",
  "gene_symbol": "AK4",
  "term_id": "GO:0004550",
  "gene": "UniProtKB:P27144",
  "gene_name": "Adenylate kinase 4, mitochondrial"
}